cellular response to vitamin A [GO:0071299] (biological process) Sources: GOC:mah Definition: Any process that results in a change in state or activity of a cell (in terms of movement, secretion, enzyme production, gene expression, etc.) as a result of a vitamin A stimulus. Also known as: cellular response to retinol Relationships: is a type of response to vitamin A [GO:0033189]; is a type of cellular response to vitamin [GO:0071295]; is a type of GO:0071396